regulation of immunoglobulin production [GO:0002637] (biological process) Relationships: is_a GO:0002700; regulates immunoglobulin production [GO:0002377] Subtypes: negative regulation of immunoglobulin production [GO:0002638], GO:0002639, regulation of isotype switching [GO:0045191], regulation of immunoglobulin production in mucosal tissue [GO:2000557] Definition: Any process that modulates the frequency, rate, or extent of immunoglobulin production. Sources: GOC:add Also known as: regulation of antibody production, regulation of immunoglobulin biosynthetic process, regulation of immunoglobulin secretion